amine biosynthetic process [GO:0009309] (biological process) Definition: The chemical reactions and pathways resulting in the formation of any organic compound that is weakly basic in character and contains an amino or a substituted amino group. Amines are called primary, secondary, or tertiary according to whether one, two, or three carbon atoms are attached to the nitrogen atom. Relationships: is a type of biosynthetic process [GO:0009058]; is a type of amine metabolic process [GO:0009308] Also known as: amine anabolism, amine biosynthesis, amine formation, amine synthesis Sources: GOC:jl, ISBN:0198506732 Subtypes: biogenic amine biosynthetic process [GO:0042401]